{
  "gene_symbol": "CCDC91",
  "gene": "UniProtKB:Q7Z6B0",
  "gene_name": "Coiled-coil domain-containing protein 91",
  "term_id": "GO:0005802",
  "term_label": "trans-Golgi network"
}